{
  "gene_name": "Apolipoprotein A-IV",
  "term_label": "very-low-density lipoprotein particle",
  "gene_symbol": "APOA4",
  "term_id": "GO:0034361",
  "gene": "UniProtKB:P06727"
}